{
  "gene_name": "PRELI domain-containing protein 2",
  "term_label": "phosphatidic acid transfer activity",
  "term_id": "GO:1990050",
  "gene_symbol": "PRELID2",
  "gene": "UniProtKB:Q8N945"
}